{
  "gene": "UniProtKB:Q9BQR3",
  "gene_name": "Serine protease 27",
  "term_label": "Unknown cellular component",
  "term_id": "UNKNOWN:0003",
  "gene_symbol": "PRSS27"
}